{
  "gene_name": "Fumarylacetoacetase",
  "gene": "UniProtKB:P16930",
  "term_id": "GO:0006559",
  "gene_symbol": "FAH",
  "term_label": "L-phenylalanine catabolic process"
}